{
  "term_label": "thioredoxin-disulfide reductase (NADPH) activity",
  "gene_name": "Thioredoxin reductase 3",
  "gene_symbol": "TXNRD3",
  "gene": "UniProtKB:Q86VQ6",
  "term_id": "GO:0004791"
}